pituitary gonadotropin complex [GO:0061696] (cellular component) Subtypes: follicle-stimulating hormone complex [GO:0016914] Relationships: is a type of protein-containing complex [GO:0032991]; is part of extracellular region [GO:0005576] References: PMID:11420129 Sources: GOC:dph Definition: A protein complex that is a protein hormone secreted by gonadotrope cells of the anterior pituitary of vertebrates. capable of regulating normal growth, sexual development, and reproductive function.